{
  "gene": "UniProtKB:Q96CV9",
  "term_label": "Golgi apparatus",
  "gene_name": "Optineurin",
  "gene_symbol": "OPTN",
  "term_id": "GO:0005794"
}